{
  "term_label": "Unknown molecular function",
  "gene": "UniProtKB:Q6ZNG2",
  "term_id": "UNKNOWN:0001",
  "gene_symbol": "DBX2",
  "gene_name": "Homeobox protein DBX2"
}